{
  "gene_name": "Homeobox protein DLX-5",
  "term_id": "GO:0030154",
  "gene_symbol": "DLX5",
  "gene": "UniProtKB:P56178",
  "term_label": "cell differentiation"
}